{
  "gene_symbol": "CCL14",
  "term_label": "inflammatory response",
  "gene": "UniProtKB:Q16627",
  "gene_name": "C-C motif chemokine 14",
  "term_id": "GO:0006954"
}